neuron differentiation involved in salivary gland development [GO:0060705] (biological process) Definition: The process in which a relatively unspecialized cell acquires specialized structural and/or functional features that characterize the neurons of the salivary gland. Sources: GOC:dph Relationships: is_a neuron differentiation [GO:0030182]; is a type of cell differentiation involved in salivary gland development [GO:0060689]